chitin-based cuticle attachment to epithelium [GO:0040005] (biological process) Definition: Attaching of a chitin-containing cuticle to the epithelium underlying it. An example of this process is found in Drosophila melanogaster. Also known as: cuticular attachment to epithelium Relationships: is a type of molting cycle process [GO:0022404]; is part of GO:0007591 Sources: GOC:bf, GOC:mtg_sensu